{
  "term_id": "UNKNOWN:0002",
  "gene": "UniProtKB:P80217",
  "gene_name": "Interferon-induced 35 kDa protein",
  "gene_symbol": "IFI35",
  "term_label": "Unknown biological process"
}